{
  "gene": "UniProtKB:Q8TE96",
  "gene_symbol": "DQX1",
  "term_label": "RNA binding",
  "term_id": "GO:0003723",
  "gene_name": "ATP-dependent RNA helicase DQX1"
}